{
  "term_id": "UNKNOWN:0003",
  "term_label": "Unknown cellular component",
  "gene_name": "TBC1 domain family member 8",
  "gene_symbol": "TBC1D8",
  "gene": "UniProtKB:O95759"
}